lateral root development [GO:0048527] (biological process) Relationships: is a type of post-embryonic root development [GO:0048528] Regulation: RO_0002212 by GO:1901332; RO_0002213 by positive regulation of lateral root development [GO:1901333]; regulated by regulation of lateral root development [GO:2000023] Sources: GOC:tb Definition: The process whose specific outcome is the progression of the lateral root over time, from its formation to the mature structure. A lateral root is one formed from pericycle cells located on the xylem radius of the root, as opposed to the initiation of the main root from the embryo proper.